{
  "gene_name": "Epithelial cell adhesion molecule",
  "term_label": "bicellular tight junction",
  "gene": "UniProtKB:P16422",
  "term_id": "GO:0005923",
  "gene_symbol": "EPCAM"
}